Pick body [GO:0097419] (cellular component) Relationships: is a type of inclusion body [GO:0016234] Sources: NIF_Subcellular:nlx_subcell_20090102 Definition: Cellular inclusion composed of numerous tau fibrils arranged in a disorderly array. Tau protein is a major component, though Pick bodies also contain ubiquitin, alpha-synuclein, and apolipoprotein E.